{
  "term_label": "glycoprotein catabolic process",
  "gene_name": "F-box only protein 17",
  "term_id": "GO:0006516",
  "gene": "UniProtKB:Q96EF6",
  "gene_symbol": "FBXO17"
}